{
  "gene": "UniProtKB:P09683",
  "gene_symbol": "SCT",
  "term_label": "negative regulation of gastrin-induced gastric acid secretion",
  "gene_name": "Secretin",
  "term_id": "GO:1903640"
}